tellurite transport [GO:0015710] (biological process) Relationships: is a type of inorganic anion transport [GO:0015698] Definition: The directed movement of tellurite into, out of or within a cell, or between cells, by means of some agent such as a transporter or pore. Sources: GOC:krc